regulation of systemic arterial blood pressure by atrial baroreceptor feedback [GO:0002015] (biological process) Relationships: is a type of heart process [GO:0003015]; is part of regulation of systemic arterial blood pressure by baroreceptor feedback [GO:0003025] Definition: A process that controls blood pressure by sensing the amount of stretch occurring in the atria. Sources: GOC:dph, GOC:tb Also known as: atrial baroreceptor regulation of systemic arterial blood pressure, atrial low pressure baroreceptor regulation of blood pressure, atrial control of blood pressure, atrial reflex